{
  "term_label": "nucleus",
  "gene_symbol": "ZCWPW1",
  "term_id": "GO:0005634",
  "gene_name": "Zinc finger CW-type PWWP domain protein 1",
  "gene": "UniProtKB:Q9H0M4"
}